protein-DNA-RNA complex assembly [GO:0001116] (biological process) Sources: GOC:txnOH Relationships: is a type of protein-DNA-RNA complex organization [GO:0001115]; is a type of protein-containing complex assembly [GO:0065003] Definition: The aggregation, arrangement and bonding together of proteins, DNA, and RNA molecules to form a protein-DNA-RNA complex.